{
  "gene_symbol": "C20orf203",
  "gene_name": "Uncharacterized protein C20orf203",
  "term_id": "UNKNOWN:0003",
  "gene": "UniProtKB:Q8NBC4",
  "term_label": "Unknown cellular component"
}